{
  "gene_name": "Intraflagellar transport protein 88 homolog",
  "gene_symbol": "IFT88",
  "gene": "UniProtKB:Q13099",
  "term_label": "non-motile cilium assembly",
  "term_id": "GO:1905515"
}